{
  "term_label": "cytokine activity",
  "gene": "UniProtKB:P09919",
  "term_id": "GO:0005125",
  "gene_symbol": "CSF3",
  "gene_name": "Granulocyte colony-stimulating factor"
}